{
  "gene": "UniProtKB:Q6V702",
  "term_label": "Unknown cellular component",
  "term_id": "UNKNOWN:0003",
  "gene_name": "Cilia- and flagella-associated protein 299",
  "gene_symbol": "CFAP299"
}